{
  "gene_name": "Probable N-acetyltransferase 16",
  "gene_symbol": "NAT16",
  "gene": "UniProtKB:Q8N8M0",
  "term_id": "UNKNOWN:0002",
  "term_label": "Unknown biological process"
}